{
  "gene": "UniProtKB:Q00535",
  "gene_symbol": "CDK5",
  "term_id": "GO:0000307",
  "gene_name": "Cyclin-dependent kinase 5",
  "term_label": "cyclin-dependent protein kinase holoenzyme complex"
}